{
  "gene_name": "Protein Flattop",
  "gene": "UniProtKB:Q5VTH2",
  "gene_symbol": "CFAP126",
  "term_label": "cilium organization",
  "term_id": "GO:0044782"
}